positive regulation of urothelial cell proliferation [GO:0050677] (biological process) Definition: Any process that activates or increases the rate or extent of urothelial cell proliferation. Sources: GOC:ai Also known as: up regulation of urothelial cell proliferation, up-regulation of urothelial cell proliferation, upregulation of urothelial cell proliferation, activation of urothelial cell proliferation, stimulation of urothelial cell proliferation Relationships: is a type of regulation of urothelial cell proliferation [GO:0050675]; is a type of positive regulation of epithelial cell proliferation [GO:0050679]; positively regulates urothelial cell proliferation [GO:0050674]